{
  "gene_symbol": "SLIT2",
  "term_id": "GO:0030308",
  "term_label": "negative regulation of cell growth",
  "gene": "UniProtKB:O94813",
  "gene_name": "Slit homolog 2 protein"
}